{
  "term_id": "GO:0005179",
  "gene": "UniProtKB:P35555",
  "gene_name": "Fibrillin-1",
  "term_label": "hormone activity",
  "gene_symbol": "FBN1"
}